{
  "term_id": "GO:0004888",
  "gene_symbol": "KIR3DS1",
  "term_label": "transmembrane signaling receptor activity",
  "gene_name": "Killer cell immunoglobulin-like receptor 3DS1",
  "gene": "UniProtKB:Q14943"
}